{
  "term_id": "UNKNOWN:0003",
  "gene_name": "Phosphatase and actin regulator 1",
  "term_label": "Unknown cellular component",
  "gene_symbol": "PHACTR1",
  "gene": "UniProtKB:Q9C0D0"
}